{
  "term_id": "UNKNOWN:0001",
  "gene": "UniProtKB:A6NK59",
  "gene_symbol": "ASB14",
  "term_label": "Unknown molecular function",
  "gene_name": "Ankyrin repeat and SOCS box protein 14"
}